{
  "term_label": "Unknown cellular component",
  "gene": "UniProtKB:P04280",
  "term_id": "UNKNOWN:0003",
  "gene_symbol": "PRB1",
  "gene_name": "Basic salivary proline-rich protein 1"
}